regulation of actin polymerization or depolymerization [GO:0008064] (biological process) Sources: GOC:mah Relationships: is_a GO:0030832; is a type of GO:0110053; RO_0002211 actin polymerization or depolymerization [GO:0008154] Definition: Any process that modulates the frequency, rate or extent of the assembly or disassembly of actin filaments by the addition or removal of actin monomers from a filament. Subtypes: regulation of actin filament polymerization [GO:0030833], regulation of actin filament depolymerization [GO:0030834]